{
  "term_label": "ubiquitin protein ligase activity",
  "gene": "UniProtKB:Q8NG27",
  "term_id": "GO:0061630",
  "gene_symbol": "PJA1",
  "gene_name": "E3 ubiquitin-protein ligase Praja-1"
}